{
  "gene_symbol": "CFAP99",
  "term_label": "Unknown cellular component",
  "gene": "UniProtKB:D6REC4",
  "term_id": "UNKNOWN:0003",
  "gene_name": "Cilia- and flagella-associated protein 99"
}